kojibiose phosphorylase activity [GO:0033831] (molecular function) Also known as: 2-alpha-D-glucosyl-D-glucose:phosphate beta-D-glucosyltransferase activity Definition: Catalysis of the reaction: kojibiose + phosphate = beta-D-glucose 1-phosphate + D-glucose. Relationships: is a type of glucosyltransferase activity [GO:0046527] Sources: EC:2.4.1.230, RHEA:11176